{
  "gene_symbol": "CYP3A7",
  "gene": "UniProtKB:P24462",
  "gene_name": "Cytochrome P450 3A7",
  "term_id": "GO:0101020",
  "term_label": "estrogen 16-alpha-hydroxylase activity"
}